{
  "term_id": "GO:0034620",
  "gene": "UniProtKB:P55061",
  "gene_name": "Bax inhibitor 1",
  "gene_symbol": "TMBIM6",
  "term_label": "cellular response to unfolded protein"
}